organomineral extracellular matrix [GO:1990377] (cellular component) Note: An example is found in shell calcitic prisms of the Mediterranean fan mussel Pinna nobilis (PMID:15994301), but the term may also be useful to annotate bone and eggshell proteins. Definition: An extracellular matrix consisting of a densely packed organomineral assembly in which the mineral phase represents the majority of the material by weight. Relationships: is a type of specialized extracellular matrix [GO:0140047] References: PMID:15994301 Sources: GOC:jh2